{
  "term_id": "UNKNOWN:0002",
  "gene_name": "Keratin-associated protein 5-6",
  "gene_symbol": "KRTAP5-6",
  "term_label": "Unknown biological process",
  "gene": "UniProtKB:Q6L8G9"
}